{
  "gene_symbol": "TPMT",
  "term_label": "Unknown biological process",
  "gene_name": "Thiopurine S-methyltransferase",
  "term_id": "UNKNOWN:0002",
  "gene": "UniProtKB:P51580"
}